{
  "gene": "UniProtKB:Q8NH63",
  "term_id": "GO:0004984",
  "term_label": "olfactory receptor activity",
  "gene_symbol": "OR51H1",
  "gene_name": "Olfactory receptor 51H1"
}